{
  "term_id": "GO:0070098",
  "gene_symbol": "CCL14",
  "gene": "UniProtKB:Q16627",
  "gene_name": "C-C motif chemokine 14",
  "term_label": "chemokine-mediated signaling pathway"
}